{
  "gene_name": "Complement factor H-related protein 5",
  "gene_symbol": "CFHR5",
  "gene": "UniProtKB:Q9BXR6",
  "term_label": "complement component C3b binding",
  "term_id": "GO:0001851"
}